{
  "term_id": "GO:0005654",
  "term_label": "nucleoplasm",
  "gene_name": "Serine_arginine-rich splicing factor 11",
  "gene_symbol": "SRSF11",
  "gene": "UniProtKB:Q05519"
}